SREBP-SCAP-Insig complex [GO:0032937] (cellular component) Definition: A protein complex formed by the association of sterol regulatory element binding protein (SREBP), SREBP-cleavage-activating protein (SCAP), and an Insig protein (Insig-1 or Insig-2) in the ER membrane. References: PMID:12923525 Relationships: is a type of membrane protein complex [GO:0098796]; is_a GO:0140534; is part of GO:0005789